{
  "term_id": "UNKNOWN:0003",
  "gene_name": "Putative zinc finger protein 730",
  "term_label": "Unknown cellular component",
  "gene_symbol": "ZNF730",
  "gene": "UniProtKB:Q6ZMV8"
}